mRNA transcription by RNA polymerase II [GO:0042789] (biological process) Sources: GOC:jl, ISBN:0321000382 Also known as: mRNA transcription from Pol II promoter, mRNA transcription from RNA polymerase II promoter Relationships: is a type of transcription by RNA polymerase II [GO:0006366]; is a type of mRNA transcription [GO:0009299] Definition: The cellular synthesis of messenger RNA (mRNA) from a DNA template by RNA polymerase II, originating at an RNA polymerase II promoter.